{
  "term_id": "UNKNOWN:0003",
  "term_label": "Unknown cellular component",
  "gene_symbol": "TRAJ1",
  "gene": "UniProtKB:A0A075B713",
  "gene_name": "T cell receptor alpha joining 1 (non-functional) (Fragment)"
}